{
  "gene_symbol": "A8MWP4",
  "gene_name": "Putative uncharacterized protein ENSP00000401716",
  "gene": "UniProtKB:A8MWP4",
  "term_label": "Unknown biological process",
  "term_id": "UNKNOWN:0002"
}